calcitonin receptor binding [GO:0031716] (molecular function) Definition: Binding to a calcitonin receptor. Sources: GOC:mah, GOC:nln Also known as: calcitonin receptor ligand Relationships: is a type of GO:0001664